septin collar [GO:0032173] (cellular component) Definition: A tubular, hourglass-shaped structure composed of highly ordered arrays of septin filaments; in budding yeast cells, the septin collar forms from the initial septin ring by expanding into the daughter cell. Relationships: is a type of septin cytoskeleton [GO:0032156]; is part of cytoskeleton [GO:0005856] Subtypes: GO:0032174, hyphae septin collar [GO:0062140] Also known as: septin hourglass References: PMID:16009555, PMID:16151244 Sources: GOC:krc